{
  "gene_name": "UPF0729 protein C18orf32",
  "gene_symbol": "C18orf32",
  "gene": "UniProtKB:Q8TCD1",
  "term_id": "UNKNOWN:0003",
  "term_label": "Unknown cellular component"
}